positive regulation of phospholipid catabolic process [GO:0060697] (biological process) Definition: Any process that increases the rate, frequency, or extent of phospholipid catabolism, the chemical reactions and pathways resulting in the breakdown of phospholipids, any lipid containing phosphoric acid as a mono- or diester. Subtypes: positive regulation of 1-phosphatidyl-1D-myo-inositol 4,5-bisphosphate catabolic process [GO:1902643], positive regulation of sphingomyelin catabolic process [GO:2000755] Sources: GOC:BHF, GOC:dph, GOC:tb Relationships: is a type of GO:0050996; is_a regulation of phospholipid catabolic process [GO:0060696]; is a type of positive regulation of phospholipid metabolic process [GO:1903727]; positively regulates phospholipid catabolic process [GO:0009395]